{
  "gene": "UniProtKB:Q14686",
  "term_label": "transcription regulator complex",
  "term_id": "GO:0005667",
  "gene_name": "Nuclear receptor coactivator 6",
  "gene_symbol": "NCOA6"
}